{
  "term_id": "GO:0005886",
  "gene": "UniProtKB:Q9H221",
  "gene_symbol": "ABCG8",
  "gene_name": "ATP-binding cassette sub-family G member 8",
  "term_label": "plasma membrane"
}